{
  "gene_name": "Keratin-associated protein 12-1",
  "term_id": "UNKNOWN:0002",
  "gene": "UniProtKB:P59990",
  "gene_symbol": "KRTAP12-1",
  "term_label": "Unknown biological process"
}